{
  "term_id": "GO:0008013",
  "term_label": "beta-catenin binding",
  "gene_symbol": "CTNNA1",
  "gene": "UniProtKB:P35221",
  "gene_name": "Catenin alpha-1"
}